{
  "gene_name": "FERM and PDZ domain-containing protein 3",
  "term_id": "UNKNOWN:0002",
  "gene_symbol": "FRMPD3",
  "term_label": "Unknown biological process",
  "gene": "UniProtKB:Q5JV73"
}